glucose fermentation to lactate and acetate [GO:0019658] (biological process) Sources: MetaCyc:P124-PWY Definition: The anaerobic chemical reactions and pathways resulting in the breakdown of glucose to lactate and acetate, yielding energy in the form of ATP. Relationships: is a type of GO:0006083; is a type of glucose catabolic process to lactate [GO:0019659]; is a type of non-glycolytic fermentation [GO:0019662] Also known as: glucose catabolic process to lactate and acetate, bifidum pathway